{
  "term_id": "GO:0016554",
  "gene": "UniProtKB:P41238",
  "term_label": "cytidine to uridine editing",
  "gene_symbol": "APOBEC1",
  "gene_name": "C-U-editing enzyme APOBEC-1"
}